{
  "gene": "UniProtKB:Q8IWV2",
  "term_label": "axon guidance",
  "term_id": "GO:0007411",
  "gene_symbol": "CNTN4",
  "gene_name": "Contactin-4"
}